{
  "gene_symbol": "PAK4",
  "term_label": "regulation of MAPK cascade",
  "gene_name": "Serine_threonine-protein kinase PAK 4",
  "term_id": "GO:0043408",
  "gene": "UniProtKB:O96013"
}